podocyte primary projection [GO:0098854] (cellular component) Relationships: is a type of plasma membrane bounded cell projection [GO:0120025] References: PMID:24309184, PMID:25324828 Definition: A cell projection originating from a renal glomerular podocyte and extending to the renal glomerular podocyte foot. Also known as: glomerular visceral epithelial cell primary projection, podocyte major process, primary podocyte process